{
  "gene_symbol": "FOXF1",
  "gene": "UniProtKB:Q12946",
  "term_id": "GO:0009887",
  "gene_name": "Forkhead box protein F1",
  "term_label": "animal organ morphogenesis"
}